{
  "term_id": "GO:0005634",
  "gene_name": "Transcription factor HIVEP3",
  "gene_symbol": "HIVEP3",
  "gene": "UniProtKB:Q5T1R4",
  "term_label": "nucleus"
}